single-stranded DNA endodeoxyribonuclease activator activity [GO:1990600] (molecular function) Definition: Increases the activity of a single-stranded DNA endodeoxyribonuclease activator activity. Relationships: is a type of GO:0140656; positively regulates GO:0000014 References: PMID:25203555